flavonol 3-O-glucosyltransferase activity [GO:0047893] (MF) Also known as: GTI, UDP-glucose flavonol 3-O-glucosyltransferase activity, UDP-glucose:flavonol 3-O-D-glucosyltransferase activity, UDP-glucose:flavonol 3-O-glucosyltransferase activity, UDPG:flavonoid-3-O-glucosyltransferase activity, UDPglucose:flavonol 3-O-D-glucosyltransferase activity, uridine diphosphoglucose-flavonol 3-O-glucosyltransferase activity Relationships: is_a GO:0035251 Definition: Catalysis of the reaction: UDP-glucose + a flavonol = UDP + a flavonol 3-O-D-glucoside. Sources: EC:2.4.1.91, MetaCyc:FLAVONOL-3-O-GLUCOSYLTRANSFERASE-RXN